{
  "gene_name": "Zinc finger protein 281",
  "gene_symbol": "ZNF281",
  "term_label": "regulation of DNA-templated transcription",
  "term_id": "GO:0006355",
  "gene": "UniProtKB:Q9Y2X9"
}